{
  "gene": "UniProtKB:O60885",
  "gene_name": "Bromodomain-containing protein 4",
  "term_id": "GO:0000785",
  "term_label": "chromatin",
  "gene_symbol": "BRD4"
}